{
  "term_label": "protein processing",
  "gene_symbol": "CPD",
  "term_id": "GO:0016485",
  "gene_name": "Carboxypeptidase D",
  "gene": "UniProtKB:O75976"
}